{
  "gene_symbol": "ILK",
  "gene": "UniProtKB:Q13418",
  "term_label": "cell-matrix adhesion",
  "gene_name": "Integrin-linked protein kinase",
  "term_id": "GO:0007160"
}